{
  "gene_name": "UDP-glucuronosyltransferase 1A9",
  "term_label": "endoplasmic reticulum",
  "gene": "UniProtKB:O60656",
  "term_id": "GO:0005783",
  "gene_symbol": "UGT1A9"
}